scaffold protein binding [GO:0097110] (molecular function) Relationships: is a type of protein binding [GO:0005515] Definition: Binding to a scaffold protein. Scaffold proteins are crucial regulators of many key signaling pathways. Although not strictly defined in function, they are known to interact and/or bind with multiple members of a signaling pathway, tethering them into complexes. References: PMID:10433269 Sources: GOC:BHF, GOC:sjp, Wikipedia:Scaffold_protein